{
  "gene_symbol": "TCAF2C",
  "term_id": "GO:0010360",
  "term_label": "negative regulation of anion channel activity",
  "gene": "UniProtKB:A0A1B0GVM2",
  "gene_name": "TRPM8 channel associated factor 2C (Fragment)"
}